{
  "gene_symbol": "MYRFL",
  "term_id": "GO:0003700",
  "gene_name": "Myelin regulatory factor-like protein",
  "term_label": "DNA-binding transcription factor activity",
  "gene": "UniProtKB:Q96LU7"
}